{
  "gene": "UniProtKB:P27169",
  "gene_name": "Serum paraoxonase_arylesterase 1",
  "term_label": "arylesterase activity",
  "gene_symbol": "PON1",
  "term_id": "GO:0004064"
}